positive regulation of toll-like receptor 11 signaling pathway [GO:0034173] (biological process) Also known as: positive regulation of TLR11 signaling pathway, positive regulation of toll-like receptor 11 signalling pathway Definition: Any process that activates or increases the frequency, rate, or extent of toll-like receptor 11 signaling pathway. Relationships: is a type of GO:0034171; is a type of positive regulation of pattern recognition receptor signaling pathway [GO:0062208]; is a type of GO:1902533; positively regulates GO:0034170 References: PMID:16551253, PMID:17328678 Sources: GOC:add